microvillar actin bundle assembly [GO:0030034] (biological process) Sources: GOC:mah Definition: Assembly of the parallel bundle of actin filaments at the core of a microvillus. Relationships: is a type of GO:0030046; is part of microvillus assembly [GO:0030033]